positive regulation of thermomorphogenesis [GO:0140922] (biological process) Relationships: is a type of positive regulation of post-embryonic development [GO:0048582]; is a type of positive regulation of response to stimulus [GO:0048584]; is a type of regulation of thermomorphogenesis [GO:0140920]; positively regulates thermomorphogenesis [GO:0140919] Definition: Any process that increases the rate, frequency or extent of thermomorphogenesis. References: PMID:27250752